{
  "term_label": "nucleus",
  "gene_name": "Signal transducer and activator of transcription 2",
  "gene_symbol": "STAT2",
  "term_id": "GO:0005634",
  "gene": "UniProtKB:P52630"
}